{
  "gene_symbol": "LAMA2",
  "term_label": "synapse",
  "term_id": "GO:0045202",
  "gene_name": "Laminin subunit alpha-2",
  "gene": "UniProtKB:P24043"
}